{
  "term_id": "GO:0006693",
  "gene": "UniProtKB:P15428",
  "gene_symbol": "HPGD",
  "term_label": "prostaglandin metabolic process",
  "gene_name": "15-hydroxyprostaglandin dehydrogenase [NAD(+)]"
}